{
  "gene_name": "Syntenin-1",
  "term_id": "GO:0005737",
  "gene_symbol": "SDCBP",
  "term_label": "cytoplasm",
  "gene": "UniProtKB:O00560"
}